{
  "gene": "UniProtKB:P48556",
  "gene_symbol": "PSMD8",
  "term_label": "proteasome regulatory particle, lid subcomplex",
  "gene_name": "26S proteasome non-ATPase regulatory subunit 8",
  "term_id": "GO:0008541"
}